{
  "term_label": "brain development",
  "term_id": "GO:0007420",
  "gene_name": "Microtubule-associated serine_threonine-protein kinase 1",
  "gene": "UniProtKB:Q9Y2H9",
  "gene_symbol": "MAST1"
}